pattern specification involved in kidney development [GO:0061004] (biological process) Also known as: kidney pattern specification, kidney pattern formation, pattern formation involved in kidney development Definition: Any developmental process that results in the creation of defined areas or spaces within the kidney to which cells respond and eventually are instructed to differentiate. Sources: GOC:dph, GOC:mtg_kidney_jan10 Relationships: is a type of pattern specification process [GO:0007389]; BFO_0000050 kidney development [GO:0001822]; BFO_0000050 renal system pattern specification [GO:0072048] Subtypes: GO:0039017, pattern specification involved in mesonephros development [GO:0061227], kidney field specification [GO:0072004], proximal/distal pattern formation involved in nephron development [GO:0072047], specification of nephron tubule identity [GO:0072081], anterior/posterior pattern specification involved in kidney development [GO:0072098], renal capsule specification [GO:0072130], pattern specification involved in metanephros development [GO:0072268]